{
  "term_id": "GO:0120009",
  "gene_symbol": "GLTPD2",
  "gene_name": "Glycolipid transfer protein domain-containing protein 2",
  "gene": "UniProtKB:A6NH11",
  "term_label": "intermembrane lipid transfer"
}